plasma membrane-derived thylakoid photosystem II [GO:0030096] (cellular component) Definition: A protein complex, located in the membrane-derived thylakoid, containing the P680 reaction center. In the light, PSII functions as a water-plastoquinone oxidoreductase, transferring electrons from water to plastoquinone. Also known as: plasma membrane photosystem II Sources: GOC:jid, GOC:mtg_sensu Relationships: is a type of photosystem II [GO:0009523]; is a type of GO:0098797; is part of cytoplasm [GO:0005737]; is part of bacterial thylakoid [GO:0030075]